{
  "gene_symbol": "TSHZ2",
  "gene": "UniProtKB:Q9NRE2",
  "term_label": "nucleus",
  "term_id": "GO:0005634",
  "gene_name": "Teashirt homolog 2"
}